regulation of leukocyte chemotaxis [GO:0002688] (biological process) Sources: GOC:add Relationships: is a type of regulation of leukocyte migration [GO:0002685]; is a type of regulation of chemotaxis [GO:0050920]; regulates leukocyte chemotaxis [GO:0030595] Also known as: regulation of immune cell chemotaxis, regulation of leucocyte chemotaxis Subtypes: negative regulation of leukocyte chemotaxis [GO:0002689], positive regulation of leukocyte chemotaxis [GO:0002690], regulation of macrophage chemotaxis [GO:0010758], GO:0060753, GO:0071622, regulation of monocyte chemotaxis [GO:0090025], regulation of lymphocyte chemotaxis [GO:1901623], regulation of dendritic cell chemotaxis [GO:2000508] Definition: Any process that modulates the frequency, rate, or extent of leukocyte chemotaxis.